{
  "term_id": "GO:0000307",
  "gene_symbol": "CDK2",
  "term_label": "cyclin-dependent protein kinase holoenzyme complex",
  "gene": "UniProtKB:P24941",
  "gene_name": "Cyclin-dependent kinase 2"
}